transport vesicle [GO:0030133] (cellular component) Definition: Any of the vesicles of the constitutive secretory pathway, which carry cargo from the endoplasmic reticulum to the Golgi, between Golgi cisternae, from the Golgi to the ER (retrograde transport) or to destinations within or outside the cell. Relationships: is a type of cytoplasmic vesicle [GO:0031410]; BFO_0000050 endomembrane system [GO:0012505] Note: Note that the term 'secretory vesicle' is sometimes used in this sense, but can also mean 'secretory granule ; GO:0030141'. Also known as: constitutive secretory pathway transport vesicle, Golgi to vacuole transport vesicle, Golgi-vacuole transport vesicle, secretory vesicle Subtypes: GO:0030140, COPI-coated Golgi to ER transport vesicle [GO:0030142], GO:0030143, clathrin-sculpted glutamate transport vesicle [GO:0060199], clathrin-sculpted acetylcholine transport vesicle [GO:0060200], GO:0070081, exocytic vesicle [GO:0070382], piccolo-bassoon transport vesicle [GO:1990257] References: PMID:22160157 Sources: GOC:mah